L(+)-lactate biosynthetic process from pyruvate [GO:0019246] (biological process) Definition: The chemical reactions and pathways resulting in the formation of L(+)-lactate from other compounds, including pyruvate. Also known as: L(+)-lactate anabolism from pyruvate, L(+)-lactate formation from pyruvate, L(+)-lactate synthesis from pyruvate, S-lactate biosynthetic process from pyruvate Relationships: is a type of lactate biosynthetic process from pyruvate [GO:0019244]; has part L-lactate dehydrogenase (NAD+) activity [GO:0004459] Sources: GOC:go_curators